{
  "term_id": "GO:0051011",
  "gene_symbol": "CAMSAP2",
  "gene_name": "Calmodulin-regulated spectrin-associated protein 2",
  "term_label": "microtubule minus-end binding",
  "gene": "UniProtKB:Q08AD1"
}